positive regulation of MHC class II biosynthetic process [GO:0045348] (biological process) Sources: GOC:go_curators Relationships: is a type of positive regulation of macromolecule biosynthetic process [GO:0010557]; is a type of regulation of MHC class II biosynthetic process [GO:0045346]; positively regulates GO:0045342 Also known as: positive regulation of MHC class II anabolism, positive regulation of MHC class II biosynthesis, positive regulation of MHC class II formation, positive regulation of MHC class II synthesis, positive regulation of major histocompatibility complex class II biosynthesis, positive regulation of major histocompatibility complex class II biosynthetic process, up regulation of MHC class II biosynthetic process, up-regulation of MHC class II biosynthetic process, upregulation of MHC class II biosynthetic process, activation of MHC class II biosynthetic process, stimulation of MHC class II biosynthetic process Definition: Any process that activates or increases the frequency, rate or extent of the chemical reactions and pathways resulting in the formation of MHC class II.